phospholipase D inhibitor activity [GO:0060961] (molecular function) Definition: Binds to and stops, prevents or reduces the activity of phospholipase D. Relationships: is a type of phospholipase inhibitor activity [GO:0004859]; negatively regulates GO:0004630 Sources: GOC:dph, GOC:tb